positive regulation of T-helper 1 cell differentiation [GO:0045627] (biological process) Sources: GOC:go_curators Note: Note that immunologists typically use the word 'development' to refer to cells of B or T cell lineages undergoing the process that GO describes as 'cell differentiation'. Also known as: up regulation of T-helper 1 cell differentiation, up-regulation of T-helper 1 cell differentiation, upregulation of T-helper 1 cell differentiation, activation of T-helper 1 cell differentiation, stimulation of T-helper 1 cell differentiation, positive regulation of T-helper 1 cell development Definition: Any process that activates or increases the frequency, rate or extent of T-helper 1 cell differentiation. Relationships: is a type of GO:0045624; is a type of regulation of T-helper 1 cell differentiation [GO:0045625]; positively regulates GO:0045063